{
  "term_label": "negative regulation of ERK1 and ERK2 cascade",
  "gene_symbol": "SPRY2",
  "term_id": "GO:0070373",
  "gene": "UniProtKB:O43597",
  "gene_name": "Protein sprouty homolog 2"
}